{
  "gene": "UniProtKB:Q9Y252",
  "gene_name": "E3 ubiquitin-protein ligase RNF6",
  "term_label": "positive regulation of DNA-templated transcription",
  "term_id": "GO:0045893",
  "gene_symbol": "RNF6"
}